{
  "gene_name": "Cdc42-interacting protein 4",
  "gene_symbol": "TRIP10",
  "gene": "UniProtKB:Q15642",
  "term_id": "UNKNOWN:0001",
  "term_label": "Unknown molecular function"
}